{
  "term_label": "cytokine receptor activity",
  "gene_name": "HLA class II histocompatibility antigen gamma chain",
  "gene": "UniProtKB:P04233",
  "term_id": "GO:0004896",
  "gene_symbol": "CD74"
}